NELF complex [GO:0032021] (cellular component) Definition: A complex of five proteins, designated NELF-A, -B, -C, -D, and -E in human, that can physically associate with RNP polymerase II to induce transcriptional pausing. References: PMID:12612062 Also known as: negative elongation factor complex Relationships: is a type of GO:0008023